{
  "gene_symbol": "OR7C2",
  "gene_name": "Olfactory receptor 7C2",
  "term_id": "GO:0004984",
  "gene": "UniProtKB:O60412",
  "term_label": "olfactory receptor activity"
}